{
  "gene_symbol": "ROCK2",
  "gene_name": "Rho-associated protein kinase 2",
  "gene": "UniProtKB:O75116",
  "term_label": "centrosome",
  "term_id": "GO:0005813"
}